{
  "gene_name": "Tripartite motif-containing protein 6",
  "gene_symbol": "TRIM6",
  "gene": "UniProtKB:Q9C030",
  "term_id": "GO:0061630",
  "term_label": "ubiquitin protein ligase activity"
}